tRNA (uracil(54)-C5)-methyltransferase activity, S-adenosyl methionine-dependent [GO:0030697] (molecular function) Also known as: RUMT, ribothymidyl synthase activity, tRNA (uracil-5-)-methyltransferase activity, S-adenosyl methionine-dependent tRNA (m5U54) methyltransferase activity, S-adenosylmethionine-dependent tRNA (m5U54) methyltransferase activity, tRNA (uracil(54)-C(5))-methyltransferase activity, S-adenosyl methionine-dependent, M5U-methyltransferase activity, RUMT activity, S-adenosyl-L-methionine:tRNA (uracil-5-)-methyltransferase activity, tRNA uracil 5-methyltransferase activity, tRNA:m(5)U54-methyltransferase activity, tRNA:m5U54-methyltransferase activity, transfer RNA uracil 5-methyltransferase activity, transfer RNA uracil methylase activity Relationships: is a type of S-adenosylmethionine-dependent methyltransferase activity [GO:0008757]; is_a tRNA (uridine) methyltransferase activity [GO:0016300] Definition: Catalysis of the reaction: S-adenosyl-L-methionine + uridine54 in tRNA = 5-methyluridine54 in tRNA + H+ + S-adenosyl-L-homocysteine. Sources: RHEA:42712